{
  "gene_name": "Alpha-synuclein",
  "term_label": "synaptic vesicle priming",
  "term_id": "GO:0016082",
  "gene_symbol": "SNCA",
  "gene": "UniProtKB:P37840"
}